{
  "gene_name": "Protein CC2D2B",
  "term_label": "non-motile cilium assembly",
  "term_id": "GO:1905515",
  "gene_symbol": "CC2D2B",
  "gene": "UniProtKB:Q6DHV5"
}